somatic recombination of immunoglobulin genes involved in immune response [GO:0002204] (BP) Definition: The process in which immunoglobulin genes are formed through recombination of the germline genetic elements, also known as immunoglobulin gene segments, within a single locus following the induction of and contributing to an immune response. Sources: GOC:add, ISBN:0781735149 Also known as: somatic recombination of antibody genes during immune response, somatic recombination of immunoglobulin genes during immune response Relationships: is a type of somatic diversification of immunoglobulins involved in immune response [GO:0002208]; is a type of somatic recombination of immunoglobulin gene segments [GO:0016447] Subtypes: GO:0045190